{
  "gene_name": "Sestrin-2",
  "term_label": "L-leucine binding",
  "term_id": "GO:0070728",
  "gene": "UniProtKB:P58004",
  "gene_symbol": "SESN2"
}